negative regulation of transforming growth factor beta production [GO:0071635] (biological process) Relationships: is a type of negative regulation of cytokine production [GO:0001818]; is_a regulation of transforming growth factor beta production [GO:0071634]; negatively regulates transforming growth factor beta production [GO:0071604] Definition: Any process that stops, prevents, or reduces the frequency, rate, or extent of production of transforming growth factor-beta. Also known as: negative regulation of TGF-B production, negative regulation of TGF-beta production, negative regulation of TGFB production, negative regulation of TGFbeta production, negative regulation of transforming growth factor-beta production, negative regulation of transforming growth factor-beta secretion Sources: GOC:mah Subtypes: GO:0032911, GO:0032912, negative regulation of transforming growth factor beta3 production [GO:0032913]